{
  "term_id": "GO:0007269",
  "gene": "UniProtKB:Q9HAP6",
  "gene_name": "Protein lin-7 homolog B",
  "gene_symbol": "LIN7B",
  "term_label": "neurotransmitter secretion"
}